{
  "gene": "UniProtKB:Q8NGQ6",
  "gene_name": "Olfactory receptor 9I1",
  "gene_symbol": "OR9I1",
  "term_id": "UNKNOWN:0003",
  "term_label": "Unknown cellular component"
}